negative regulation of cytolysis [GO:0045918] (biological process) Definition: Any process that stops, prevents, or reduces the frequency, rate or extent of cytolysis. Relationships: is a type of regulation of cytolysis [GO:0042268]; is a type of negative regulation of cellular process [GO:0048523]; negatively regulates cytolysis [GO:0019835] Sources: GOC:go_curators Also known as: down regulation of cytolysis, down-regulation of cytolysis, downregulation of cytolysis, inhibition of cytolysis